acyl-CoA desaturase activity [GO:0016215] (molecular function) Also known as: CoA desaturase activity Definition: Catalysis of the reaction: acyl-CoA + reduced acceptor + O2 = desaturated-acyl-CoA + acceptor + 2 H2O. Subtypes: stearoyl-CoA 9-desaturase activity [GO:0004768], acyl-CoA 6-desaturase activity [GO:0016213], acyl-CoA 11-(Z)-desaturase activity [GO:0017105], palmitoyl-CoA 9-desaturase activity [GO:0032896], acyl-CoA 11-(E)-desaturase activity [GO:0050600], acyl-CoA (8-3)-desaturase activity [GO:0062076], acyl-CoA (9+3)-desaturase activity [GO:0102985], acyl-CoA 15-desaturase activity [GO:0102988] Relationships: is a type of oxidoreductase activity, acting on paired donors, with oxidation of a pair of donors resulting in the reduction of molecular oxygen to two molecules of water [GO:0016717] References: PMID:36017969